syntaxin binding [GO:0019905] (molecular function) Sources: ISBN:0198506732 Subtypes: syntaxin-1 binding [GO:0017075], syntaxin-3 binding [GO:0030348] Also known as: syntaxin-13 binding, syntaxin-2 binding, syntaxin-5 binding, syntaxin-6 binding Definition: Binding to a syntaxin, a SNAP receptor involved in the docking of synaptic vesicles at the presynaptic zone of a synapse. Relationships: is a type of SNARE binding [GO:0000149]